regulation of receptor signaling pathway via JAK-STAT [GO:0046425] (biological process) Relationships: is a type of regulation of receptor signaling pathway via STAT [GO:1904892]; regulates cell surface receptor signaling pathway via JAK-STAT [GO:0007259] Also known as: STAT protein import into nucleus, regulation of STAT protein import into nucleus, regulation of STAT protein nuclear translocation Subtypes: negative regulation of receptor signaling pathway via JAK-STAT [GO:0046426], positive regulation of receptor signaling pathway via JAK-STAT [GO:0046427] Definition: Any process that modulates the frequency, rate or extent of receptor signaling via JAK-STAT. Sources: GOC:bf